{
  "term_id": "GO:0046513",
  "gene": "UniProtKB:Q6ZMG9",
  "gene_symbol": "CERS6",
  "gene_name": "Ceramide synthase 6",
  "term_label": "ceramide biosynthetic process"
}